{
  "gene": "UniProtKB:Q9Y490",
  "term_id": "GO:0005737",
  "term_label": "cytoplasm",
  "gene_name": "Talin-1",
  "gene_symbol": "TLN1"
}